response to salt stress [GO:0009651] (biological process) Also known as: response to ionic osmotic stress, salinity response Relationships: is a type of response to osmotic stress [GO:0006970] Definition: Any process that results in a change in state or activity of a cell or an organism (in terms of movement, secretion, enzyme production, gene expression, etc.) as a result of a stimulus indicating an increase or decrease in the concentration of salt (particularly but not exclusively sodium and chloride ions) in the environment. Sources: GOC:jl Subtypes: GO:0042538, hypotonic salinity response [GO:0042539], GO:0043157, cellular response to salt stress [GO:0071472], GO:0072342 Regulation: regulated by GO:1901000; negatively regulated by GO:1901001; positively regulated by positive regulation of response to salt stress [GO:1901002]